{
  "gene": "UniProtKB:A6NCJ1",
  "term_label": "Unknown biological process",
  "gene_symbol": "TEKTIP1",
  "gene_name": "Tektin bundle-interacting protein 1",
  "term_id": "UNKNOWN:0002"
}